{
  "gene": "UniProtKB:Q53S58",
  "gene_name": "Transmembrane protein 177",
  "gene_symbol": "TMEM177",
  "term_label": "Unknown molecular function",
  "term_id": "UNKNOWN:0001"
}